{
  "term_id": "UNKNOWN:0001",
  "gene_name": "Mesoderm-specific transcript homolog protein",
  "gene": "UniProtKB:Q5EB52",
  "term_label": "Unknown molecular function",
  "gene_symbol": "MEST"
}